{
  "term_label": "Unknown cellular component",
  "gene_symbol": "NHSL3",
  "gene": "UniProtKB:Q9P206",
  "gene_name": "Uncharacterized protein KIAA1522",
  "term_id": "UNKNOWN:0003"
}